{
  "term_id": "GO:0051480",
  "gene_name": "Short transient receptor potential channel 5",
  "gene": "UniProtKB:Q9UL62",
  "gene_symbol": "TRPC5",
  "term_label": "regulation of cytosolic calcium ion concentration"
}